{
  "gene_name": "Serine_threonine-protein kinase B-raf",
  "term_id": "GO:0000165",
  "term_label": "MAPK cascade",
  "gene": "UniProtKB:P15056",
  "gene_symbol": "BRAF"
}